{
  "term_label": "ubiquitin-like ligase-substrate adaptor activity",
  "gene_symbol": "KLHL10",
  "gene": "UniProtKB:Q6JEL2",
  "term_id": "GO:1990756",
  "gene_name": "Kelch-like protein 10"
}